{
  "term_label": "Unknown cellular component",
  "gene_name": "Protein kinase C iota type",
  "gene_symbol": "PRKCI",
  "term_id": "UNKNOWN:0003",
  "gene": "UniProtKB:P41743"
}